{
  "term_id": "UNKNOWN:0003",
  "gene_symbol": "OR5F1",
  "gene": "UniProtKB:O95221",
  "gene_name": "Olfactory receptor 5F1",
  "term_label": "Unknown cellular component"
}